negative regulation of translational initiation in response to osmotic stress [GO:0032063] (biological process) Definition: Any process that stops, prevents or reduces the rate of translation initiation, as a result of a stimulus indicating an increase or decrease in the concentration of solutes outside the organism or cell. Also known as: down regulation of translation initiation in response to osmotic stress, down-regulation of translation initiation in response to osmotic stress, downregulation of translation initiation in response to osmotic stress, inhibition of translation initiation in response to osmotic stress Sources: GOC:mah Relationships: is a type of GO:0032057; is a type of negative regulation of translation in response to osmotic stress [GO:0032061]; is a type of regulation of translational initiation in response to osmotic stress [GO:0043561]